{
  "term_id": "GO:0022857",
  "gene": "UniProtKB:Q9UGQ3",
  "gene_symbol": "SLC2A6",
  "term_label": "transmembrane transporter activity",
  "gene_name": "Solute carrier family 2, facilitated glucose transporter member 6"
}